{
  "gene": "UniProtKB:Q8WVM7",
  "gene_name": "Cohesin subunit SA-1",
  "term_id": "GO:0007062",
  "term_label": "sister chromatid cohesion",
  "gene_symbol": "STAG1"
}